{
  "term_id": "GO:0005518",
  "term_label": "collagen binding",
  "gene": "UniProtKB:Q92791",
  "gene_symbol": "P3H4",
  "gene_name": "Endoplasmic reticulum protein SC65"
}